Ndc80 complex [GO:0031262] (cellular component) References: PMID:28502666, PMID:34810257 Sources: GOC:vw Also known as: Nuf2-Ndc80 complex Definition: An essential outer kinetochore complex involved in the attachment of microtubule ends to the chromosomes during mitosis. Relationships: is a type of protein-containing complex [GO:0032991]; is part of outer kinetochore [GO:0000940]